{
  "gene_name": "Putative serine_threonine-protein phosphatase 4 regulatory subunit 1-like",
  "term_id": "UNKNOWN:0002",
  "term_label": "Unknown biological process",
  "gene": "UniProtKB:Q9P1A2",
  "gene_symbol": "PPP4R1L"
}